{
  "gene": "UniProtKB:Q96LB9",
  "gene_symbol": "PGLYRP3",
  "term_label": "N-acetylmuramoyl-L-alanine amidase activity",
  "gene_name": "Peptidoglycan recognition protein 3",
  "term_id": "GO:0008745"
}